{
  "gene": "UniProtKB:Q8WXG6",
  "term_label": "regulation of apoptotic process",
  "term_id": "GO:0042981",
  "gene_symbol": "MADD",
  "gene_name": "MAP kinase-activating death domain protein"
}